{
  "term_label": "Unknown cellular component",
  "gene_symbol": "ZNF621",
  "gene_name": "Zinc finger protein 621",
  "gene": "UniProtKB:Q6ZSS3",
  "term_id": "UNKNOWN:0003"
}